{
  "gene": "UniProtKB:Q9UN88",
  "term_label": "synaptic transmission, GABAergic",
  "gene_name": "Gamma-aminobutyric acid receptor subunit theta",
  "gene_symbol": "GABRQ",
  "term_id": "GO:0051932"
}